RNA 3'-end processing [GO:0031123] (biological process) Definition: Any process involved in forming the mature 3' end of an RNA molecule. Also known as: RNA 3' end processing Sources: GOC:mah Relationships: is a type of RNA processing [GO:0006396] Subtypes: mitochondrial RNA 3'-end processing [GO:0000965], mRNA 3'-end processing [GO:0031124], GO:0031125, sno(s)RNA 3'-end processing [GO:0031126], snRNA 3'-end processing [GO:0034472], tRNA 3'-end processing [GO:0042780], regulatory ncRNA 3'-end processing [GO:0043628], co-transcriptional RNA 3'-end processing, cleavage and polyadenylation pathway [GO:0180012]